{
  "gene_symbol": "KCNIP2",
  "gene_name": "Kv channel-interacting protein 2",
  "gene": "UniProtKB:Q9NS61",
  "term_label": "regulation of potassium ion transmembrane transport",
  "term_id": "GO:1901379"
}